{
  "gene": "UniProtKB:Q9UBK9",
  "gene_symbol": "UXT",
  "gene_name": "Protein UXT",
  "term_label": "chromatin",
  "term_id": "GO:0000785"
}